peptidyl-alanine modification [GO:0018194] (biological process) Relationships: is a type of peptidyl-amino acid modification [GO:0018193] Sources: GOC:go_curators Definition: The modification of peptidyl-alanine. Subtypes: N-terminal peptidyl-alanine methylation [GO:0018011], peptidyl-D-alanine racemization [GO:0019122]